{
  "term_id": "GO:0070847",
  "term_label": "core mediator complex",
  "gene_name": "Mediator of RNA polymerase II transcription subunit 8",
  "gene": "UniProtKB:Q96G25",
  "gene_symbol": "MED8"
}